{
  "gene_symbol": "PF4V1",
  "gene_name": "Platelet factor 4 variant",
  "term_id": "GO:0006954",
  "term_label": "inflammatory response",
  "gene": "UniProtKB:P10720"
}